{
  "gene_name": "Zinc finger protein 382",
  "term_label": "RNA polymerase II cis-regulatory region sequence-specific DNA binding",
  "gene": "UniProtKB:Q96SR6",
  "gene_symbol": "ZNF382",
  "term_id": "GO:0000978"
}